{
  "gene_name": "FHF complex subunit HOOK interacting protein 2A",
  "gene_symbol": "FHIP2A",
  "term_id": "UNKNOWN:0001",
  "gene": "UniProtKB:Q5W0V3",
  "term_label": "Unknown molecular function"
}